positive regulation of methanofuran biosynthetic process [GO:1900353] (biological process) Relationships: is a type of GO:0009891; is_a GO:1900351; positively regulates methanofuran biosynthetic process [GO:2001120] Definition: Any process that activates or increases the frequency, rate or extent of methanofuran biosynthetic process. Sources: GOC:TermGenie, GOC:mengo_curators Also known as: activation of methanofuran biosynthesis, positive regulation of methanofuran biosynthesis, up regulation of methanofuran biosynthesis, up regulation of methanofuran biosynthetic process, up-regulation of methanofuran biosynthesis, up-regulation of methanofuran biosynthetic process, upregulation of methanofuran biosynthesis, upregulation of methanofuran biosynthetic process, activation of methanofuran biosynthetic process